{
  "term_label": "cytoplasm",
  "term_id": "GO:0005737",
  "gene_symbol": "AGO1",
  "gene_name": "Protein argonaute-1",
  "gene": "UniProtKB:Q9UL18"
}